{
  "gene_symbol": "KCNN3",
  "gene": "UniProtKB:Q9UGI6",
  "gene_name": "Small conductance calcium-activated potassium channel protein 3",
  "term_label": "potassium ion transmembrane transport",
  "term_id": "GO:0071805"
}